{
  "gene": "UniProtKB:O75864",
  "term_id": "UNKNOWN:0001",
  "term_label": "Unknown molecular function",
  "gene_symbol": "PPP1R37",
  "gene_name": "Protein phosphatase 1 regulatory subunit 37"
}